{
  "gene": "UniProtKB:Q1L6U9",
  "gene_name": "Prostate-associated microseminoprotein",
  "term_label": "Unknown biological process",
  "term_id": "UNKNOWN:0002",
  "gene_symbol": "MSMP"
}